{
  "gene_name": "Fanconi anemia group G protein",
  "term_id": "GO:0043240",
  "term_label": "Fanconi anaemia nuclear complex",
  "gene_symbol": "FANCG",
  "gene": "UniProtKB:O15287"
}